peptidyl-glutamic acid modification [GO:0018200] (biological process) Subtypes: peptidyl-glutamic acid carboxylation [GO:0017187], N-terminal peptidyl-glutamic acid acetylation [GO:0018002], GO:0018094, protein polyglutamylation [GO:0018095], nickel incorporation into iron-sulfur cluster via tris-L-cysteinyl L-cysteine persulfido L-glutamato L-histidino L-serinyl nickel triiron disulfide trioxide [GO:0018418], protein deglutamylation [GO:0035608] Sources: GOC:go_curators Definition: The modification of peptidyl-glutamic acid. Relationships: is a type of peptidyl-amino acid modification [GO:0018193]